positive regulation of cell fate commitment [GO:0010455] (biological process) Sources: GOC:dph, GOC:tb Definition: Any process that activates, maintains or increases the frequency or rate of cell fate commitment. Cell fate commitment is the commitment of cells to specific cell fates and their capacity to differentiate into particular kinds of cells. Positional information is established through protein signals that emanate from a localized source within a cell (the initial one-cell zygote) or within a developmental field. Subtypes: GO:0042660, GO:0060225, positive regulation of R7 cell fate commitment [GO:0106397], positive regulation of T-helper 17 cell lineage commitment [GO:2000330], positive regulation of venous endothelial cell fate commitment [GO:2000789] Relationships: is a type of regulation of cell fate commitment [GO:0010453]; is a type of positive regulation of cell differentiation [GO:0045597]; positively regulates cell fate commitment [GO:0045165]